{
  "term_label": "regulation of ventricular cardiac muscle cell membrane repolarization",
  "gene": "UniProtKB:P15382",
  "gene_name": "Potassium voltage-gated channel subfamily E member 1",
  "gene_symbol": "KCNE1",
  "term_id": "GO:0060307"
}